L-lysine import across plasma membrane [GO:0097639] (biological process) Regulation: regulated by regulation of L-lysine import across plasma membrane [GO:1905008]; negatively regulated by negative regulation of L-lysine import across plasma membrane [GO:1905009]; positively regulated by positive regulation of L-lysine import across plasma membrane [GO:1905010] Also known as: L-lysine import into cell Definition: The directed movement of L-lysine from outside of a cell, across the plasma membrane and into the cytosol. References: PMID:8195186 Sources: GOC:krc Relationships: is a type of amino acid import across plasma membrane [GO:0089718]; is a type of L-lysine transmembrane transport [GO:1903401]